{
  "term_label": "Unknown biological process",
  "gene_symbol": "KRBA1",
  "gene_name": "Protein KRBA1",
  "term_id": "UNKNOWN:0002",
  "gene": "UniProtKB:A5PL33"
}